{
  "gene_symbol": "TMEM167A",
  "term_label": "Unknown cellular component",
  "gene": "UniProtKB:Q8TBQ9",
  "term_id": "UNKNOWN:0003",
  "gene_name": "Protein kish-A"
}